{
  "gene_symbol": "AMH",
  "gene": "UniProtKB:P03971",
  "term_id": "GO:0001880",
  "term_label": "Mullerian duct regression",
  "gene_name": "Muellerian-inhibiting factor"
}